{
  "gene_symbol": "DAW1",
  "term_label": "ubiquitin-like ligase-substrate adaptor activity",
  "gene": "UniProtKB:Q8N136",
  "term_id": "GO:1990756",
  "gene_name": "Dynein assembly factor with WDR repeat domains 1"
}